polyphosphate kinase complex [GO:0009358] (cellular component) Note: See also the molecular function term 'polyphosphate kinase activity ; GO:0008976'. Sources: GOC:mah Definition: A protein complex that possesses polyphosphate kinase activity. Relationships: is a type of GO:0061695